NAD-dependent protein depalmitoylase activity [GO:0140774] (molecular function) Definition: Catalysis of the reaction: N6-octadecanoyl-L-lysyl-[protein] + NAD+ + H2O = octadecanoyl-ADP-D-ribose + L-lysyl-[protein] + nicotinamide. References: PMID:23552949 Sources: RHEA:70563 Relationships: is a type of acyltransferase activity, transferring groups other than amino-acyl groups [GO:0016747]; is part of GO:0043687